regulation of G2/MI transition of meiotic cell cycle [GO:0110030] (biological process) Sources: GOC:vw Relationships: is a type of regulation of meiotic cell cycle phase transition [GO:1901993]; is a type of regulation of cell cycle G2/M phase transition [GO:1902749]; regulates G2/MI transition of meiotic cell cycle [GO:0008315] Subtypes: negative regulation of G2/MI transition of meiotic cell cycle [GO:0110031], positive regulation of G2/MI transition of meiotic cell cycle [GO:0110032] Definition: Any signaling pathway that modulates the activity of a cell cycle cyclin-dependent protein kinase to modulate the switch from G2 phase to MI phase of the meiotic cell cycle.